regulation of complement activation [GO:0030449] (biological process) Subtypes: regulation of complement activation, lectin pathway [GO:0001868], regulation of activation of membrane attack complex [GO:0001969], regulation of complement activation, classical pathway [GO:0030450], regulation of complement activation, alternative pathway [GO:0030451], GO:0045916, GO:0045917 Relationships: is a type of regulation of immune effector process [GO:0002697]; is a type of regulation of humoral immune response [GO:0002920]; regulates complement activation [GO:0006956] Sources: GOC:go_curators Also known as: regulation of complement cascade Definition: Any process that modulates the frequency, rate or extent of complement activation.